{
  "gene_symbol": "PLEKHM1",
  "term_label": "Unknown biological process",
  "gene_name": "Pleckstrin homology domain-containing family M member 1",
  "gene": "UniProtKB:Q9Y4G2",
  "term_id": "UNKNOWN:0002"
}